{
  "gene": "UniProtKB:Q5VSL9",
  "gene_name": "Striatin-interacting protein 1",
  "gene_symbol": "STRIP1",
  "term_id": "GO:0030674",
  "term_label": "protein-macromolecule adaptor activity"
}